{
  "gene_name": "Immunoglobulin superfamily member 21",
  "term_label": "plasma membrane",
  "gene": "UniProtKB:Q96ID5",
  "gene_symbol": "IGSF21",
  "term_id": "GO:0005886"
}